MPF complex [GO:0031387] (cellular component) Definition: A complex consisting of a Cdc2-class (also known as Cdc28) cyclin-dependent kinase and an M-phase cyclin such as S. pombe Cdc13. The MPF complex phosphorylates and activates the anaphase promoting complex (APC). Relationships: is a type of GO:0000307 References: PMID:12045216